{
  "gene": "UniProtKB:Q01860",
  "term_label": "RNA polymerase II cis-regulatory region sequence-specific DNA binding",
  "term_id": "GO:0000978",
  "gene_symbol": "POU5F1",
  "gene_name": "POU domain, class 5, transcription factor 1"
}